{
  "term_label": "cholesterol binding",
  "term_id": "GO:0015485",
  "gene_name": "Oxysterol-binding protein-related protein 8",
  "gene": "UniProtKB:Q9BZF1",
  "gene_symbol": "OSBPL8"
}